{
  "gene": "UniProtKB:P28838",
  "gene_symbol": "LAP3",
  "term_label": "peptidase activity",
  "term_id": "GO:0008233",
  "gene_name": "Cytosol aminopeptidase"
}